{
  "term_id": "GO:0015116",
  "term_label": "sulfate transmembrane transporter activity",
  "gene_name": "Anion exchange transporter",
  "gene": "UniProtKB:Q8TE54",
  "gene_symbol": "SLC26A7"
}